{
  "gene": "UniProtKB:P17181",
  "gene_symbol": "IFNAR1",
  "term_label": "type I interferon-mediated signaling pathway",
  "term_id": "GO:0060337",
  "gene_name": "Interferon alpha_beta receptor 1"
}